male germline ring canal [GO:0035323] (cellular component) Relationships: is a type of germline ring canal [GO:0045172] References: PMID:9635420 Also known as: spermatocyte ring canal, testicular ring canal Definition: An intercellular bridge that connects the germline cells of a male cyst.